{
  "gene_symbol": "SPATA7",
  "term_label": "photoreceptor distal connecting cilium",
  "gene_name": "Spermatogenesis-associated protein 7",
  "term_id": "GO:0120206",
  "gene": "UniProtKB:Q9P0W8"
}